{
  "gene": "UniProtKB:O95819",
  "term_id": "GO:0048812",
  "term_label": "neuron projection morphogenesis",
  "gene_name": "Mitogen-activated protein kinase kinase kinase kinase 4",
  "gene_symbol": "MAP4K4"
}